{
  "gene_name": "Estrogen receptor",
  "gene_symbol": "ESR1",
  "term_id": "GO:0071391",
  "term_label": "cellular response to estrogen stimulus",
  "gene": "UniProtKB:P03372"
}